{
  "term_label": "molecular adaptor activity",
  "gene_symbol": "FIS1",
  "term_id": "GO:0060090",
  "gene_name": "Mitochondrial fission 1 protein",
  "gene": "UniProtKB:Q9Y3D6"
}